{
  "term_label": "negative regulation of transcription by RNA polymerase II",
  "gene_name": "Non-structural maintenance of chromosomes element 3 homolog",
  "term_id": "GO:0000122",
  "gene": "UniProtKB:Q96MG7",
  "gene_symbol": "NSMCE3"
}